{
  "gene": "UniProtKB:Q7Z6M1",
  "gene_symbol": "RABEPK",
  "gene_name": "Rab9 effector protein with kelch motifs",
  "term_id": "UNKNOWN:0002",
  "term_label": "Unknown biological process"
}